{
  "gene_symbol": "REM1",
  "gene": "UniProtKB:O75628",
  "term_id": "GO:0005246",
  "gene_name": "GTP-binding protein REM 1",
  "term_label": "calcium channel regulator activity"
}